primary palate development [GO:1903929] (biological process) Definition: The process whose specific outcome is the progression of a primary palate over time, from its formation to the mature structure. References: PMID:24644145, PMID:25504820 Sources: GOC:TermGenie, GOC:mgi_curators, GO_REF:0000094 Also known as: primary palate process development, palatum primarium development, primitive palate development, processus palatinus medianus development Relationships: is a type of roof of mouth development [GO:0060021]